{
  "gene_name": "PIH1 domain-containing protein 2",
  "gene_symbol": "PIH1D2",
  "term_id": "GO:0006364",
  "term_label": "rRNA processing",
  "gene": "UniProtKB:Q8WWB5"
}